cellular response to vasopressin [GO:1904117] (biological process) Definition: Any process that results in a change in state or activity of a cell (in terms of movement, secretion, enzyme production, gene expression, etc.) as a result of a vasopressin stimulus. Relationships: is a type of cellular response to peptide hormone stimulus [GO:0071375]; is a type of response to vasopressin [GO:1904116] References: PMID:22811487 Sources: GOC:TermGenie, GO_REF:0000071